{
  "term_label": "nucleus",
  "gene_name": "Tudor-interacting repair regulator protein",
  "gene_symbol": "NUDT16L1",
  "gene": "UniProtKB:Q9BRJ7",
  "term_id": "GO:0005634"
}